regulation of sporangium development [GO:0075310] (biological process) Definition: Any process that modulates the frequency, rate or extent of sporangium development, a process that leads to the formation of sporangium, a single-celled or many-celled structure in which spores are produced, as in fungi, algae, mosses, and ferns, gymnosperms, angiosperms. Subtypes: regulation of sporangium germination [GO:0075223], GO:0075311, negative regulation of sporangium development [GO:0075312], regulation of oomycete sporangium development [GO:0075322] Sources: GOC:pamgo_curators Relationships: is a type of regulation of spore-bearing organ development [GO:0075260]; regulates sporangium development [GO:0043582]